{
  "gene_symbol": "IGFBPL1",
  "term_id": "GO:0005615",
  "gene_name": "Insulin-like growth factor-binding protein-like 1",
  "term_label": "extracellular space",
  "gene": "UniProtKB:Q8WX77"
}